oxidoreductase activity, acting on paired donors, with incorporation or reduction of molecular oxygen, reduced ascorbate as one donor, and incorporation of one atom of oxygen [GO:0016715] (molecular function) Relationships: is a type of monooxygenase activity [GO:0004497]; is a type of oxidoreductase activity, acting on paired donors, with incorporation or reduction of molecular oxygen [GO:0016705] Sources: EC:1.14.17.- Subtypes: dopamine beta-monooxygenase activity [GO:0004500], peptidylglycine monooxygenase activity [GO:0004504], tyramine-beta hydroxylase activity [GO:0004836], 1-aminocyclopropane-1-carboxylate oxidase activity [GO:0009815] Definition: Catalysis of an oxidation-reduction (redox) reaction in which hydrogen or electrons are transferred from reduced ascorbate and one other donor, and one atom of oxygen is incorporated into one donor.